{
  "gene": "UniProtKB:Q13137",
  "gene_name": "Calcium-binding and coiled-coil domain-containing protein 2",
  "term_id": "GO:0098792",
  "gene_symbol": "CALCOCO2",
  "term_label": "xenophagy"
}